ATPase inhibitor complex [GO:1903503] (cellular component) References: PMID:16170325 Sources: GOC:TermGenie, GOC:bhm, GO_REF:0000088 Subtypes: exon-exon junction subcomplex mago-y14 [GO:1990501] Note: An example of this is Mago in drome (P49028) in PMID:16170325 (inferred from direct assay). Relationships: is a type of protein-containing complex [GO:0032991] Definition: A protein complex which is capable of ATPase inhibitor activity.